protein localization to paranode region of axon [GO:0002175] (biological process) Relationships: is a type of protein localization to axon [GO:0099612] References: PMID:18803321 Definition: A cellular protein localization process in which a protein is transported to, or maintained at, the paranode region of an axon. Also known as: protein localisation to paranode region of axon